cyclic nucleotide-activated monoatomic ion channel activity [GO:0043855] (molecular function) Subtypes: intracellularly cyclic nucleotide-activated monoatomic cation channel activity [GO:0005221] Relationships: is a type of GO:0015276 Definition: Enables the transmembrane transfer of an ion by a channel that opens when a cyclic nucleotide has been bound by the channel complex or one of its constituent parts. Sources: GOC:jl Regulation: regulated by GO:1902159 Also known as: cyclic nucleotide-gated ion channel activity, cyclic nucleotide activated ion channel activity, cyclic nucleotide gated ion channel activity, cyclic nucleotide-gated monoatomic ion channel activity